interleukin-23-mediated signaling pathway [GO:0038155] (biological process) Relationships: is a type of GO:0019221 Definition: The series of molecular signals initiated by interleukin-23 binding to its receptor on the surface of a target cell, and ending with the regulation of a downstream cellular process, e.g. transcription. Also known as: IL-23-mediated signaling pathway, interleukin-23-mediated signalling pathway Sources: GOC:nhn, GOC:signaling